{
  "gene_name": "Alpha-taxilin",
  "gene": "UniProtKB:P40222",
  "term_label": "Unknown biological process",
  "term_id": "UNKNOWN:0002",
  "gene_symbol": "TXLNA"
}